{
  "term_id": "GO:0016139",
  "gene_name": "Tissue alpha-L-fucosidase",
  "gene_symbol": "FUCA1",
  "gene": "UniProtKB:P04066",
  "term_label": "glycoside catabolic process"
}